{
  "gene": "UniProtKB:Q9HBE5",
  "term_label": "cytokine-mediated signaling pathway",
  "term_id": "GO:0019221",
  "gene_name": "Interleukin-21 receptor",
  "gene_symbol": "IL21R"
}